{
  "gene_name": "F-actin-capping protein subunit alpha-3",
  "gene": "UniProtKB:Q96KX2",
  "gene_symbol": "CAPZA3",
  "term_label": "actin cytoskeleton organization",
  "term_id": "GO:0030036"
}